{
  "gene_name": "Zinc finger protein 485",
  "gene": "UniProtKB:Q8NCK3",
  "term_id": "GO:0005634",
  "gene_symbol": "ZNF485",
  "term_label": "nucleus"
}